root epidermal cell differentiation [GO:0010053] (biological process) Sources: GOC:tb Definition: The process in which a relatively unspecialized cell in the root epidermis acquires the specialized features of a trichoblast or atrichoblast. Subtypes: trichoblast differentiation [GO:0010054], GO:0010055, GO:0048765 Relationships: is a type of plant epidermal cell differentiation [GO:0090627]; is part of root morphogenesis [GO:0010015]; is part of GO:0090558